{
  "gene_name": "snRNA-activating protein complex subunit 5",
  "gene": "UniProtKB:O75971",
  "gene_symbol": "SNAPC5",
  "term_label": "Unknown biological process",
  "term_id": "UNKNOWN:0002"
}